{
  "gene_name": "Putative olfactory receptor 1F2",
  "term_id": "GO:0004984",
  "gene": "UniProtKB:Q96R84",
  "gene_symbol": "OR1F2P",
  "term_label": "olfactory receptor activity"
}